{
  "term_id": "GO:0005829",
  "gene_symbol": "PLA2G4B",
  "term_label": "cytosol",
  "gene": "UniProtKB:P0C869",
  "gene_name": "Cytosolic phospholipase A2 beta"
}